cellular anatomical entity morphogenesis [GO:0032989] (biological process) Relationships: is a type of cellular component organization [GO:0016043] Sources: GOC:dph, GOC:mah, GOC:tb Also known as: cellular component morphogenesis, cellular structure morphogenesis Definition: The process in which a cellular entity is generated and organized. A cellular entity has granularity above the level of a protein complex but below that of an anatomical system.